{
  "gene_name": "Putative protein SSX9",
  "term_label": "nucleus",
  "gene_symbol": "SSX9P",
  "term_id": "GO:0005634",
  "gene": "UniProtKB:Q7RTT3"
}